cellular response to heparin [GO:0071504] (biological process) Relationships: is a type of response to heparin [GO:0071503]; is_a GO:1901699; is a type of cellular response to oxygen-containing compound [GO:1901701] Definition: Any process that results in a change in state or activity of a cell (in terms of movement, secretion, enzyme production, gene expression, etc.) as a result of a heparin stimulus. Sources: GOC:mah, GOC:yaf